{
  "term_label": "U4 snRNA 3'-end processing",
  "gene": "UniProtKB:Q9NQT5",
  "gene_symbol": "EXOSC3",
  "gene_name": "Exosome complex component RRP40",
  "term_id": "GO:0034475"
}